{
  "gene_name": "Mu-type opioid receptor",
  "term_id": "GO:0001965",
  "term_label": "G-protein alpha-subunit binding",
  "gene": "UniProtKB:P35372",
  "gene_symbol": "OPRM1"
}